mammary gland cord formation [GO:0060616] (biological process) Relationships: is a type of GO:0016331; is a type of epithelial tube formation [GO:0072175]; is part of mammary gland cord morphogenesis [GO:0060652] References: PMID:12558599 Sources: GOC:dph Definition: The process in which the mammary gland cord forms by elongation of the mammary bud. The cord is formed once the elongating bud breaks through the mesenchyme and reaches the fat pad. Also known as: mammary gland sprout formation